{
  "gene": "UniProtKB:Q8NH18",
  "gene_symbol": "OR5J2",
  "term_id": "UNKNOWN:0002",
  "gene_name": "Olfactory receptor 5J2",
  "term_label": "Unknown biological process"
}